cullin-RING ubiquitin ligase complex [GO:0031461] (cellular component) References: PMID:15571813, PMID:15688063 Relationships: is a type of ubiquitin ligase complex [GO:0000151] Subtypes: anaphase-promoting complex [GO:0005680], SCF ubiquitin ligase complex [GO:0019005], Cul2-RING ubiquitin ligase complex [GO:0031462], Cul3-RING ubiquitin ligase complex [GO:0031463], GO:0031466, Cul7-RING ubiquitin ligase complex [GO:0031467], Cul8-RING ubiquitin ligase complex [GO:0035361], Cul4-RING E3 ubiquitin ligase complex [GO:0080008] Also known as: CRL complex, cullin complex, cullin-RING ligase Definition: Any ubiquitin ligase complex in which the catalytic core consists of a member of the cullin family and a RING domain protein; the core is associated with one or more additional proteins that confer substrate specificity.